{
  "gene_name": "mRNA cap guanine-N7 methyltransferase",
  "term_label": "nucleus",
  "term_id": "GO:0005634",
  "gene_symbol": "RNMT",
  "gene": "UniProtKB:O43148"
}